non-motile cilium assembly [GO:1905515] (biological process) References: PMID:14521833, PMID:14521834 Sources: GOC:TermGenie, GOC:cilia, GOC:kmv, GO_REF:0000079 Regulation: regulated by regulation of non-motile cilium assembly [GO:1902855]; negatively regulated by negative regulation of non-motile cilium assembly [GO:1902856]; positively regulated by positive regulation of non-motile cilium assembly [GO:1902857] Relationships: is_a cilium assembly [GO:0060271] Definition: The aggregation, arrangement and bonding together of a set of components to form a non-motile cilium. Also known as: non-motile cilium formation, nonmotile cilium assembly, nonmotile cilium formation, immotile primary cilium assembly, nonmotile primary cilia assembly, nonmotile primary cilium assembly, sensory cilium assembly, sensory cilium biogenesis